calcium-activated cation channel activity [GO:0005227] (molecular function) Also known as: calcium activated cation channel activity, intracellular calcium-activated potassium channel, polycystin Definition: Enables the transmembrane transfer of an inorganic cation by a channel that opens when a calcium cation has been bound by the channel complex or one of its constituent parts. Relationships: is a type of GO:0022839; is a type of ligand-gated monoatomic cation channel activity [GO:0099094] Sources: GOC:dph, GOC:mtg_transport Subtypes: calcium-activated potassium channel activity [GO:0015269]